mitotic checkpoint complex, CDC20-MAD2 subcomplex [GO:1990333] (cellular component) Definition: A protein complex involved in the spindle checkpoint, preventing the activation of the anaphase-promoting complex until all chromosomes are correctly attached in a bipolar fashion to the mitotic spindle. In budding yeast this complex consists of Mad2p and Cdc20p, and in mammalian cells it consists of MAD2 and CDC20. Note: An example of this is cdc20 in Saccharomyces cerevisiae (P26309) in PMID:15879521 (inferred from direct assay). Also known as: CDC20-MAD2 complex Relationships: is a type of GO:0140513; is part of mitotic checkpoint complex [GO:0033597] References: PMID:15879521 Sources: GOC:bhm